prostaglandin catabolic process [GO:1905344] (biological process) References: PMID:25290914 Sources: GOC:BHF, GOC:TermGenie, GOC:rl, GO_REF:0000068 Also known as: prostaglandin breakdown, prostaglandin catabolism, prostaglandin degradation Regulation: regulated by regulation of prostaglandin catabolic process [GO:1905828]; negatively regulated by negative regulation of prostaglandin catabolic process [GO:1905829]; positively regulated by GO:1905830 Relationships: is a type of prostanoid catabolic process [GO:0062232] Definition: The chemical reactions and pathways resulting in the breakdown of prostaglandin.